neuromast regeneration [GO:0070657] (biological process) References: PMID:19381250 Sources: GOC:dsf Definition: The regrowth of a neuromast following its loss or destruction. Relationships: is a type of mechanosensory epithelium regeneration [GO:0070655]